{
  "term_label": "endoplasmic reticulum",
  "term_id": "GO:0005783",
  "gene": "UniProtKB:P13667",
  "gene_name": "Protein disulfide-isomerase A4",
  "gene_symbol": "PDIA4"
}